{
  "term_id": "GO:0005739",
  "gene_symbol": "SLC25A45",
  "term_label": "mitochondrion",
  "gene": "UniProtKB:Q8N413",
  "gene_name": "Solute carrier family 25 member 45"
}